{
  "term_label": "Unknown molecular function",
  "gene_symbol": "LINC00305",
  "gene": "UniProtKB:Q7Z4B0",
  "gene_name": "Putative uncharacterized protein encoded by LINC00305",
  "term_id": "UNKNOWN:0001"
}